{
  "term_label": "endosome",
  "gene_name": "AP-1 complex-associated regulatory protein",
  "gene_symbol": "AP1AR",
  "gene": "UniProtKB:Q63HQ0",
  "term_id": "GO:0005768"
}